{
  "gene_name": "Zinc finger protein 62 homolog",
  "term_label": "nucleus",
  "gene_symbol": "ZFP62",
  "gene": "UniProtKB:Q8NB50",
  "term_id": "GO:0005634"
}